positive regulation of glutathione biosynthetic process [GO:1903788] (biological process) Definition: Any process that activates or increases the frequency, rate or extent of glutathione biosynthetic process. Sources: GOC:PARL, GOC:TermGenie, GOC:bf, GO_REF:0000058 Relationships: is a type of positive regulation of biosynthetic process [GO:0009891]; is a type of positive regulation of amide metabolic process [GO:0034250]; is a type of regulation of glutathione biosynthetic process [GO:1903786]; positively regulates glutathione biosynthetic process [GO:0006750] Also known as: positive regulation of glutathione anabolism, positive regulation of glutathione biosynthesis, positive regulation of glutathione formation, positive regulation of glutathione synthesis, up regulation of glutathione anabolism, up regulation of glutathione biosynthesis, up regulation of glutathione biosynthetic process, up regulation of glutathione formation, up regulation of glutathione synthesis, up-regulation of glutathione anabolism, up-regulation of glutathione biosynthesis, up-regulation of glutathione biosynthetic process, up-regulation of glutathione formation, up-regulation of glutathione synthesis, upregulation of glutathione anabolism, upregulation of glutathione biosynthesis, upregulation of glutathione biosynthetic process, upregulation of glutathione formation, upregulation of glutathione synthesis, activation of glutathione anabolism, activation of glutathione biosynthesis, activation of glutathione biosynthetic process, activation of glutathione formation, activation of glutathione synthesis